benzodiazepine receptor binding [GO:0030156] (MF) Relationships: is_a signaling receptor binding [GO:0005102] References: PMID:9915832 Sources: GOC:ceb, GOC:mah Also known as: benzodiazepine receptor ligand, diazepam binding inhibitor activity Definition: Binding to a peripheral benzodiazepine receptor (PBR).